{
  "term_label": "photoreceptor outer segment",
  "gene_symbol": "OPN1SW",
  "gene_name": "Short-wave-sensitive opsin 1",
  "gene": "UniProtKB:P03999",
  "term_id": "GO:0001750"
}